{
  "gene_name": "Rho GTPase-activating protein 45",
  "gene": "UniProtKB:Q92619",
  "gene_symbol": "ARHGAP45",
  "term_id": "GO:0016020",
  "term_label": "membrane"
}